{
  "gene": "UniProtKB:Q96P63",
  "term_label": "Unknown biological process",
  "gene_name": "Serpin B12",
  "term_id": "UNKNOWN:0002",
  "gene_symbol": "SERPINB12"
}